{
  "term_id": "GO:0007186",
  "gene_name": "Adhesion G protein-coupled receptor L1",
  "gene_symbol": "ADGRL1",
  "gene": "UniProtKB:O94910",
  "term_label": "G protein-coupled receptor signaling pathway"
}